extracellular matrix-dependent thymocyte migration [GO:0072680] (biological process) References: PMID:20856819 Sources: CL:0000893, GOC:BHF, GOC:mah Definition: The movement of a thymocyte through distinct intrathymic niches (e.g. medulla, cortex), where it receives a unique set of developmental cues required for T-cell development, dependent on extracellular matrix components including fibronectin, collagen and laminin. Also known as: extracellular matrix-dependent thymic lymphocyte migration, extracellular matrix-dependent immature T cell migration, extracellular matrix-dependent immature T lymphocyte migration, extracellular matrix-dependent immature T-cell migration, extracellular matrix-dependent immature T-lymphocyte migration Relationships: is a type of substrate-dependent cell migration [GO:0006929]; is a type of thymocyte migration [GO:0072679] Subtypes: fibronectin-dependent thymocyte migration [GO:0072681]